{
  "gene": "UniProtKB:Q9Y2Z4",
  "term_label": "cytosol",
  "gene_name": "Tyrosine--tRNA ligase, mitochondrial",
  "gene_symbol": "YARS2",
  "term_id": "GO:0005829"
}